{
  "gene_name": "Down syndrome critical region protein 8",
  "term_label": "Unknown biological process",
  "term_id": "UNKNOWN:0002",
  "gene_symbol": "DSCR8",
  "gene": "UniProtKB:Q96T75"
}